negative regulation of canonical Wnt signaling pathway [GO:0090090] (biological process) Also known as: negative regulation of Wnt receptor signaling pathway through beta-catenin, negative regulation of canonical Wnt receptor signaling pathway, negative regulation of canonical Wnt receptor signalling pathway, negative regulation of canonical Wnt-activated signaling pathway, negative regulation of catenin import into nucleus, negative regulation of catenin protein nuclear translocation Sources: GOC:dph, GOC:tb Definition: Any process that decreases the rate, frequency, or extent of the Wnt signaling pathway through beta-catenin, the series of molecular signals initiated by binding of a Wnt protein to a frizzled family receptor on the surface of the target cell, followed by propagation of the signal via beta-catenin, and ending with a change in transcription of target genes. Relationships: is a type of GO:0030178; is a type of GO:0060828; negatively regulates canonical Wnt signaling pathway [GO:0060070]